detection of hexose stimulus [GO:0009732] (biological process) Definition: The series of events in which a stimulus from a hexose is received and converted into a molecular signal. Sources: GOC:sm Relationships: is a type of response to hexose [GO:0009746]; is a type of detection of monosaccharide stimulus [GO:0034287] Subtypes: detection of glucose [GO:0051594] Also known as: perception of hexose stimulus